{
  "gene_symbol": "TOR1B",
  "term_id": "GO:0005635",
  "term_label": "nuclear envelope",
  "gene_name": "Torsin-1B",
  "gene": "UniProtKB:O14657"
}